{
  "gene": "UniProtKB:Q9UP65",
  "term_id": "GO:0047498",
  "gene_symbol": "PLA2G4C",
  "term_label": "calcium-dependent phospholipase A2 activity",
  "gene_name": "Cytosolic phospholipase A2 gamma"
}